{
  "term_id": "GO:0005634",
  "term_label": "nucleus",
  "gene_symbol": "KDM1A",
  "gene": "UniProtKB:O60341",
  "gene_name": "Lysine-specific histone demethylase 1A"
}